THPH synthase activity [GO:0106265] (molecular function) Also known as: polyketide syntase Definition: Catalysis of the reaction: 3 H+ + hexanoyl-CoA + 3 malonyl-CoA = 2,4,6-trihydroxyphenylhexan-1-one + 3 CO2 + 4 CoA. References: PMID:9446571 Sources: RHEA:64352 Relationships: is a type of transferase activity [GO:0016740]